{
  "gene_name": "Disks large homolog 2",
  "gene": "UniProtKB:Q15700",
  "term_id": "GO:0098839",
  "gene_symbol": "DLG2",
  "term_label": "postsynaptic density membrane"
}